{
  "gene_name": "CTD small phosphatase-like protein 2",
  "gene": "UniProtKB:Q05D32",
  "term_id": "UNKNOWN:0002",
  "term_label": "Unknown biological process",
  "gene_symbol": "CTDSPL2"
}